{
  "gene_symbol": "DCLRE1C",
  "gene": "UniProtKB:Q96SD1",
  "term_id": "GO:0070419",
  "gene_name": "Protein artemis",
  "term_label": "nonhomologous end joining complex"
}